{
  "term_label": "Unknown biological process",
  "gene_name": "NIF3-like protein 1",
  "term_id": "UNKNOWN:0002",
  "gene_symbol": "NIF3L1",
  "gene": "UniProtKB:Q9GZT8"
}